interleukin-2 receptor complex [GO:0005893] (cellular component) Also known as: IL-2 receptor complex Relationships: is a type of plasma membrane signaling receptor complex [GO:0098802] References: PMID:3116143, PMID:8266078 Sources: GOC:mah Definition: A protein complex that binds interleukin-2; comprises alpha, beta, and gamma subunits.